negative regulation of protein glutathionylation [GO:0010734] (biological process) Definition: Any process that decreases the rate, frequency, or extent of protein glutathionylation. Protein glutathionylation is the protein modification process in which a glutathione molecule is added to a protein amino acid through a disulfide linkage. Sources: GOC:BHF, GOC:dph, GOC:rl, GOC:tb Relationships: is a type of regulation of protein glutathionylation [GO:0010732]; is a type of negative regulation of protein modification process [GO:0031400]; RO_0002212 protein glutathionylation [GO:0010731] Also known as: negative regulation of protein amino acid glutathionylation